protein insertion into mitochondrial outer membrane [GO:0045040] (biological process) Relationships: is a type of outer mitochondrial membrane organization [GO:0007008]; is a type of protein insertion into mitochondrial membrane [GO:0051204] Regulation: regulated by regulation of protein insertion into mitochondrial outer membrane [GO:1903636]; negatively regulated by GO:1903637; positively regulated by positive regulation of protein insertion into mitochondrial outer membrane [GO:1903638] Definition: The process comprising the insertion of proteins from outside the organelle into the mitochondrial outer membrane, mediated by large outer membrane translocase complexes. Also known as: mitochondrial outer membrane protein import, protein import into mitochondrial outer membrane, protein transport into mitochondrial outer membrane References: PMID:18672008 Sources: GOC:mcc, GOC:vw